{
  "gene_symbol": "FOXO4",
  "gene_name": "Forkhead box protein O4",
  "gene": "UniProtKB:P98177",
  "term_label": "RNA polymerase II cis-regulatory region sequence-specific DNA binding",
  "term_id": "GO:0000978"
}